{
  "gene": "UniProtKB:P21673",
  "gene_symbol": "SAT1",
  "gene_name": "Diamine acetyltransferase 1",
  "term_id": "UNKNOWN:0003",
  "term_label": "Unknown cellular component"
}